{
  "gene_symbol": "INSL6",
  "gene_name": "Insulin-like peptide INSL6",
  "gene": "UniProtKB:Q9Y581",
  "term_label": "Unknown biological process",
  "term_id": "UNKNOWN:0002"
}